response to interleukin-1 [GO:0070555] (biological process) Definition: Any process that results in a change in state or activity of a cell or an organism (in terms of movement, secretion, enzyme production, gene expression, etc.) as a result of an interleukin-1 stimulus. Subtypes: GO:0071347 Also known as: response to IL-1 Sources: GOC:BHF, GOC:mah Relationships: is a type of response to cytokine [GO:0034097]